{
  "term_id": "UNKNOWN:0003",
  "gene": "UniProtKB:C9JTQ0",
  "gene_name": "Ankyrin repeat domain-containing protein 63",
  "gene_symbol": "ANKRD63",
  "term_label": "Unknown cellular component"
}